p-hydroxyphenyl lignin catabolic process [GO:1901059] (biological process) Also known as: H-lignin catabolic process, p-hydroxyphenyl lignin breakdown, p-hydroxyphenyl lignin catabolism, p-hydroxyphenyl lignin degradation Relationships: is_a lignin catabolic process [GO:0046274] Sources: GOC:TermGenie, GOC:mengo_curators Definition: The chemical reactions and pathways resulting in the breakdown of p-hydroxyphenyl lignin.